{
  "gene": "UniProtKB:Q8TE69",
  "gene_symbol": "EOLA1",
  "term_id": "UNKNOWN:0001",
  "term_label": "Unknown molecular function",
  "gene_name": "Protein EOLA1"
}